{
  "gene_symbol": "FUT3",
  "term_id": "UNKNOWN:0003",
  "gene": "UniProtKB:P21217",
  "gene_name": "3-galactosyl-N-acetylglucosaminide 4-alpha-L-fucosyltransferase FUT3",
  "term_label": "Unknown cellular component"
}